negative regulation of meiotic joint molecule formation [GO:0010947] (biological process) Relationships: is a type of regulation of meiotic joint molecule formation [GO:0010946]; is a type of negative regulation of cell cycle process [GO:0010948]; is a type of GO:2000242; negatively regulates meiotic joint molecule formation [GO:0000709] Definition: Any process that decreases the frequency, rate or extent of meiotic joint molecule formation. Meiotic joint molecule formation is the conversion of the paired broken DNA and homologous duplex DNA into a four-stranded branched intermediate, known as a joint molecule, formed during meiotic recombination. Sources: GOC:dph, GOC:tb